{
  "gene_symbol": "CLEC1A",
  "term_label": "signal transduction",
  "gene_name": "C-type lectin domain family 1 member A",
  "term_id": "GO:0007165",
  "gene": "UniProtKB:Q8NC01"
}